{
  "term_id": "GO:0005743",
  "term_label": "mitochondrial inner membrane",
  "gene_symbol": "NOA1",
  "gene": "UniProtKB:Q8NC60",
  "gene_name": "Nitric oxide-associated protein 1"
}